positive regulation of fast-twitch skeletal muscle fiber contraction [GO:0031448] (biological process) Relationships: is a type of regulation of fast-twitch skeletal muscle fiber contraction [GO:0031446]; is a type of positive regulation of striated muscle contraction [GO:0045989]; positively regulates fast-twitch skeletal muscle fiber contraction [GO:0031443] Definition: Any process that activates or increases the frequency, rate or extent of fast-twitch skeletal muscle contraction. Also known as: positive regulation of fast-twitch skeletal muscle contraction, up regulation of fast-twitch skeletal muscle contraction, up-regulation of fast-twitch skeletal muscle contraction, upregulation of fast-twitch skeletal muscle contraction, activation of fast-twitch skeletal muscle contraction, stimulation of fast-twitch skeletal muscle contraction Sources: GOC:dph, GOC:ef, GOC:mah, GOC:mtg_muscle, GOC:tb